positive regulation of transcription from RNA polymerase II promoter by glucose [GO:0000432] (biological process) Relationships: is a type of regulation of transcription from RNA polymerase II promoter by glucose [GO:0000430]; is_a carbon catabolite activation of transcription from RNA polymerase II promoter [GO:0000436]; is a type of positive regulation of transcription by glucose [GO:0046016] Also known as: up regulation of transcription from RNA polymerase II promoter by glucose, up-regulation of transcription from RNA polymerase II promoter by glucose, upregulation of transcription from RNA polymerase II promoter by glucose, activation of transcription from RNA polymerase II promoter by glucose, stimulation of transcription from RNA polymerase II promoter by glucose Sources: GOC:krc Definition: Any process involving glucose that activates or increases the rate of transcription from an RNA polymerase II promoter.